proton transmembrane transporter activity [GO:0015078] (molecular function) Relationships: is a type of monoatomic cation transmembrane transporter activity [GO:0008324]; is part of GO:1902600 Also known as: hydrogen ion transmembrane transporter activity, proton transporter activity Subtypes: GO:0000514, cytochrome-c oxidase activity [GO:0004129], acetylcholine:proton antiporter activity [GO:0005278], quinol-cytochrome-c reductase activity [GO:0008121], NADH dehydrogenase (ubiquinone) activity [GO:0008137], GO:0008553, GO:0008750, GO:0009678, proton channel activity [GO:0015252], solute:proton symporter activity [GO:0015295], cycloheximide:proton antiporter activity [GO:0015309], benomyl:proton antiporter activity [GO:0015310], monoamine:proton antiporter activity [GO:0015311], polyamine:proton antiporter activity [GO:0015312], tetracycline:proton antiporter activity [GO:0015520], acridine:proton antiporter activity [GO:0042962], azole:proton antiporter activity [GO:0045119], proton-transporting ATPase activity, rotational mechanism [GO:0046961], GO:0051139, chloride:proton antiporter activity [GO:0062158], GO:0106421, L-alanine:proton antiporter activity [GO:0140407], glycine:proton antiporter activity [GO:0140799], gamma-aminobutyric acid:proton antiporter activity [GO:0140800], polyspecific organic cation:proton antiporter activity [GO:0140968] Sources: GOC:ai Definition: Enables the transfer of a proton from one side of a membrane to the other.